{
  "gene": "UniProtKB:Q9GZT6",
  "term_label": "mitochondrion",
  "gene_name": "Coiled-coil domain-containing protein 90B, mitochondrial",
  "term_id": "GO:0005739",
  "gene_symbol": "CCDC90B"
}